{
  "term_label": "positive regulation of transcription by RNA polymerase II",
  "gene_name": "Myocyte-specific enhancer factor 2A",
  "gene": "UniProtKB:Q02078",
  "term_id": "GO:0045944",
  "gene_symbol": "MEF2A"
}